{
  "gene_symbol": "ORC3",
  "gene_name": "Origin recognition complex subunit 3",
  "term_id": "GO:0006270",
  "term_label": "DNA replication initiation",
  "gene": "UniProtKB:Q9UBD5"
}